N-acetylglucosamine-6-sulfatase activity [GO:0008449] (molecular function) Also known as: chondroitinsulfatase, N-acetylglucosamine-6-sulphatase activity, 2-acetamido-2-deoxy-D-glucose 6-sulfate sulfatase activity, N-acetyl-D-glucosamine-6-sulfate 6-sulfohydrolase activity, N-acetylglucosamine 6-sulfate sulfatase activity, O,N-disulfate O-sulfohydrolase activity, acetylglucosamine 6-sulfatase activity, glucosamine-6-sulfatase activity Relationships: is a type of sulfuric ester hydrolase activity [GO:0008484] Sources: EC:3.1.6.14 Definition: Catalysis of the hydrolysis of the 6-sulfate group of the N-acetyl-D-glucosamine 6-sulfate units of heparan sulfate and keratan sulfate.